{
  "gene_symbol": "ZNG1A",
  "gene_name": "Zinc-regulated GTPase metalloprotein activator 1A",
  "term_id": "GO:0005737",
  "gene": "UniProtKB:Q9BRT8",
  "term_label": "cytoplasm"
}